{
  "gene": "UniProtKB:O75592",
  "term_label": "ubiquitin protein ligase activity",
  "term_id": "GO:0061630",
  "gene_name": "E3 ubiquitin-protein ligase MYCBP2",
  "gene_symbol": "MYCBP2"
}